{
  "term_id": "UNKNOWN:0002",
  "term_label": "Unknown biological process",
  "gene_symbol": "TRMT2A",
  "gene_name": "tRNA (uracil-5-)-methyltransferase homolog A",
  "gene": "UniProtKB:Q8IZ69"
}